extrinsic component of nuclear outer membrane [GO:0031316] (cellular component) Definition: The component of a nuclear outer membrane consisting of gene products and protein complexes that are loosely bound to one of its surfaces, but not integrated into the hydrophobic region. Sources: GOC:dos, GOC:mah Also known as: extrinsic to nuclear outer membrane Relationships: is a type of extrinsic component of organelle membrane [GO:0031312]; is part of GO:0005640